trans-synaptic signaling by trans-synaptic complex [GO:0099545] (biological process) Sources: GOC:dos Subtypes: GO:0098941, retrograde trans-synaptic signaling by trans-synaptic protein complex [GO:0098942], trans-synaptic signaling by trans-synaptic complex, modulating synaptic transmission [GO:0099557] Relationships: is a type of trans-synaptic signaling [GO:0099537] Definition: Cell-cell signaling between presynapse and postsynapse mediated by a trans-synaptic protein complex.